regulation of age-related resistance [GO:1904248] (BP) References: PMID:19694953 Sources: GOC:TermGenie, GO_REF:0000058 Relationships: is a type of regulation of innate immune response [GO:0045088]; is a type of regulation of developmental process [GO:0050793]; regulates age-related resistance [GO:0090644] Subtypes: negative regulation of age-related resistance [GO:1904249], positive regulation of age-related resistance [GO:1904250] Definition: Any process that modulates the extent of age-related resistance. Also known as: regulation of developmental resistance, regulation of ontogenic resistance, regulation of ARR, regulation of adult seedling resistance, regulation of flowering-induced resistance, regulation of mature seedling resistance, regulation of senescence-induced resistance